regulation of adipose tissue development [GO:1904177] (biological process) References: PMID:23081848 Sources: GOC:TermGenie, GO_REF:0000058 Also known as: regulation of adipogenesis Definition: Any process that modulates the frequency, rate or extent of adipose tissue development. Subtypes: GO:1904178, positive regulation of adipose tissue development [GO:1904179] Relationships: is a type of regulation of developmental process [GO:0050793]; regulates adipose tissue development [GO:0060612]